{
  "gene": "UniProtKB:P51523",
  "term_id": "UNKNOWN:0003",
  "term_label": "Unknown cellular component",
  "gene_name": "Zinc finger protein 84",
  "gene_symbol": "ZNF84"
}